{
  "gene": "UniProtKB:A0A1B0GWI6",
  "term_id": "UNKNOWN:0002",
  "gene_name": "Uncharacterized protein",
  "term_label": "Unknown biological process",
  "gene_symbol": "LOC101059915"
}